negative regulation of meiotic chromosome separation [GO:1905133] (biological process) Definition: Any process that stops, prevents or reduces the frequency, rate or extent of meiotic chromosome separation. Relationships: is a type of regulation of meiotic chromosome separation [GO:1905132]; is a type of GO:1905819; is a type of negative regulation of reproductive process [GO:2000242]; negatively regulates meiotic chromosome separation [GO:0051307] References: PMID:15620645 Sources: GOC:TermGenie, GOC:vw, GO_REF:0000058 Subtypes: negative regulation of metaphase/anaphase transition of meiotic cell cycle [GO:1902103] Also known as: down regulation of chromosome separation during meiosis, down regulation of meiotic chromosome resolution, down regulation of meiotic chromosome separation, down-regulation of chromosome separation during meiosis, down-regulation of meiotic chromosome resolution, down-regulation of meiotic chromosome separation, downregulation of chromosome separation during meiosis, downregulation of meiotic chromosome resolution, downregulation of meiotic chromosome separation, negative regulation of chromosome separation during meiosis, negative regulation of meiotic chromosome resolution, inhibition of chromosome separation during meiosis, inhibition of meiotic chromosome resolution, inhibition of meiotic chromosome separation